{
  "gene_symbol": "GRIN2D",
  "term_label": "transmitter-gated monoatomic ion channel activity involved in regulation of postsynaptic membrane potential",
  "term_id": "GO:1904315",
  "gene": "UniProtKB:O15399",
  "gene_name": "Glutamate receptor ionotropic, NMDA 2D"
}